{
  "gene_name": "Leucine repeat adapter protein 25",
  "gene": "UniProtKB:Q8N5H3",
  "term_label": "transcription corepressor binding",
  "gene_symbol": "FAM89B",
  "term_id": "GO:0001222"
}